{
  "gene": "UniProtKB:P62266",
  "gene_symbol": "RPS23",
  "term_id": "GO:0003735",
  "term_label": "structural constituent of ribosome",
  "gene_name": "Small ribosomal subunit protein uS12"
}